dihydrolipoyllysine-residue succinyltransferase activity [GO:0004149] (molecular function) Definition: Catalysis of the reaction: N(6)-[(R)-dihydrolipoyl]-L-lysyl-[2-oxoglutarate dehydrogenase complex component E2] + succinyl-CoA = N(6)-[(R)-S(8)-succinyldihydrolipoyl]-L-lysyl-[2-oxoglutarate dehydrogenase complex component E2] + CoA. Relationships: is a type of S-succinyltransferase activity [GO:0016751]; is a type of catalytic activity, acting on a protein [GO:0140096] Sources: RHEA:15213 Also known as: dihydrolipoamide S-succinyltransferase activity, dihydrolipoamide succinyltransferase activity, dihydrolipoic transsuccinylase activity, dihydrolipolyl transsuccinylase activity, dihydrolipoyl transsuccinylase activity, enzyme-dihydrolipoyllysine:succinyl-CoA S-succinyltransferase activity, lipoate succinyltransferase (Escherichia coli) activity, lipoate succinyltransferase activity, lipoic transsuccinylase activity, lipoyl transsuccinylase activity, succinyl-CoA:dihydrolipoamide S-succinyltransferase activity, succinyl-CoA:dihydrolipoate S-succinyltransferase activity, succinyl-CoA:enzyme-6-N-(dihydrolipoyl)lysine S-succinyltransferase activity, succinyl-CoA:enzyme-N6-(dihydrolipoyl)lysine S-succinyltransferase activity